{
  "gene": "UniProtKB:O75326",
  "gene_name": "Semaphorin-7A",
  "term_id": "GO:0030215",
  "gene_symbol": "SEMA7A",
  "term_label": "semaphorin receptor binding"
}